{
  "term_id": "UNKNOWN:0002",
  "gene": "UniProtKB:Q5T5S1",
  "gene_name": "Coiled-coil domain-containing protein 183",
  "gene_symbol": "CCDC183",
  "term_label": "Unknown biological process"
}